{
  "term_label": "Golgi cis cisterna",
  "gene_symbol": "GOLGA2",
  "gene_name": "Golgin subfamily A member 2",
  "gene": "UniProtKB:Q08379",
  "term_id": "GO:0000137"
}